Derlin-1 retrotranslocation complex [GO:0036513] (cellular component) Relationships: is a type of GO:0098796; is a type of GO:0140534; is part of endoplasmic reticulum membrane [GO:0005789] Definition: A protein complex that functions in the retrotranslocation step of ERAD (ER-associated protein degradation), and includes at its core Derlin-1 oligomers forming a retrotranslocation channel. References: PMID:15215856, PMID:16186510 Sources: GOC:PARL, GOC:bf Note: The Derlin-1 retrotranslocation complex is likely to assemble in steps, thereby containing different components at different stages of the retrotranslocation process. Also known as: Derlin-1 complex, Derlin-1 protein dislocation complex, Derlin-1 retro-translocation complex, Derlin-1 retrotranslocon, ERAD protein dislocation complex